{
  "term_id": "UNKNOWN:0001",
  "gene": "UniProtKB:Q17R55",
  "term_label": "Unknown molecular function",
  "gene_symbol": "FAM187B",
  "gene_name": "Protein FAM187B"
}